{
  "gene_symbol": "GOLGA6L1",
  "gene_name": "Golgin subfamily A member 6-like protein 1",
  "term_label": "Unknown cellular component",
  "term_id": "UNKNOWN:0003",
  "gene": "UniProtKB:Q8N7Z2"
}